{
  "gene_symbol": "SHANK1",
  "gene_name": "SH3 and multiple ankyrin repeat domains protein 1",
  "term_id": "GO:0043197",
  "gene": "UniProtKB:Q9Y566",
  "term_label": "dendritic spine"
}